histone H1-4S187 kinase activity [GO:0140191] (molecular function) References: PMID:21511733 Relationships: is a type of protein serine/threonine kinase activity [GO:0004674]; is a type of histone H1 kinase activity [GO:0140190] Definition: Catalysis of the reaction: histone H1-4-serine (position 27) + ATP = histone H1-4-phosphoserine (position 27) + ADP.